{
  "term_id": "UNKNOWN:0002",
  "gene_symbol": "RLN3",
  "term_label": "Unknown biological process",
  "gene_name": "Relaxin-3",
  "gene": "UniProtKB:Q8WXF3"
}